sulfolipid metabolic process [GO:0046505] (biological process) References: PMID:9751667 Definition: The chemical reactions and pathways involving sulfolipids, any compound containing a sulfonic acid residue joined by a carbon-sulfur bond to a lipid. Relationships: is a type of lipid metabolic process [GO:0006629]; is a type of sulfur compound metabolic process [GO:0006790] Subtypes: sulfolipid biosynthetic process [GO:0046506] Also known as: sulfolipid metabolism, sulpholipid metabolic process, sulpholipid metabolism